{
  "term_label": "cell-cell signaling",
  "gene_name": "Four-jointed box protein 1",
  "gene_symbol": "FJX1",
  "gene": "UniProtKB:Q86VR8",
  "term_id": "GO:0007267"
}